{
  "term_label": "Unknown cellular component",
  "gene_symbol": "SLC7A11",
  "gene": "UniProtKB:Q9UPY5",
  "term_id": "UNKNOWN:0003",
  "gene_name": "Cystine_glutamate transporter"
}